palmitoleyl hydrolase activity [GO:1990699] (molecular function) References: PMID:25731175 Definition: Catalysis of a hydrolase reaction that removes a palmitoleyl moiety, a 16-carbon monounsaturated fatty acid (C16:1), from some substrate. Relationships: is a type of carboxylic ester hydrolase activity [GO:0052689]